{
  "gene_name": "Glycophorin-A",
  "gene": "UniProtKB:P02724",
  "gene_symbol": "GYPA",
  "term_id": "UNKNOWN:0002",
  "term_label": "Unknown biological process"
}